{
  "gene_symbol": "MLEC",
  "term_label": "Unknown biological process",
  "term_id": "UNKNOWN:0002",
  "gene_name": "Malectin",
  "gene": "UniProtKB:Q14165"
}